calcitonin family receptor complex [GO:1903439] (cellular component) Definition: A protein complex which is capable of calcitonin family receptor activity. Calcitonin family receptors may form dimers, trimers or tetramers; adrenomedullin and amylin receptors have only been observed as dimers so far. Subtypes: adrenomedullin receptor complex [GO:1903143], amylin receptor complex [GO:1903440], CGRP receptor complex [GO:1990406] References: PMID:10871296, PMID:12037140, PMID:18687416 Sources: GOC:TermGenie, GOC:bhm, GO_REF:0000088 Relationships: is a type of G protein-coupled receptor complex [GO:0097648]